{
  "gene_name": "Solute carrier organic anion transporter family member 2A1",
  "term_id": "GO:0016323",
  "gene": "UniProtKB:Q92959",
  "gene_symbol": "SLCO2A1",
  "term_label": "basolateral plasma membrane"
}